{
  "gene_name": "Small ribosomal subunit protein uS2",
  "gene_symbol": "RPSA",
  "term_id": "GO:0002181",
  "gene": "UniProtKB:P08865",
  "term_label": "cytoplasmic translation"
}